serine-tRNA ligase activity [GO:0004828] (molecular function) Definition: Catalysis of the reaction: ATP + L-serine + tRNA(Ser) = AMP + diphosphate + L-seryl-tRNA(Ser). Also catalyzes the formation of L-seryl-tRNA(Sec) from tRNA(Sec), the special tRNA for selenocysteine. Also known as: seryl-tRNA synthetase activity, L-serine:tRNASer ligase (AMP-forming), SerRS activity, serine translase activity, seryl-transfer RNA synthetase activity, seryl-transfer ribonucleate synthetase activity, seryl-transfer ribonucleic acid synthetase activity Relationships: is a type of aminoacyl-tRNA ligase activity [GO:0004812] Sources: EC:6.1.1.11